{
  "gene": "UniProtKB:Q7Z7L1",
  "gene_name": "Schlafen family member 11",
  "term_id": "GO:0051607",
  "term_label": "defense response to virus",
  "gene_symbol": "SLFN11"
}